{
  "gene": "UniProtKB:P35498",
  "gene_symbol": "SCN1A",
  "term_id": "GO:0086002",
  "term_label": "cardiac muscle cell action potential involved in contraction",
  "gene_name": "Sodium channel protein type 1 subunit alpha"
}